{
  "gene": "UniProtKB:Q99879",
  "term_label": "antibacterial humoral response",
  "gene_name": "Histone H2B type 1-M",
  "gene_symbol": "H2BC14",
  "term_id": "GO:0019731"
}